positive regulation of phosphorelay signal transduction system [GO:0070299] (BP) Relationships: is a type of regulation of phosphorelay signal transduction system [GO:0070297]; is a type of positive regulation of intracellular signal transduction [GO:1902533]; positively regulates phosphorelay signal transduction system [GO:0000160] Definition: Any process that activates or increases the frequency, rate or extent of signal transduction via a phosphorelay signal transduction system. Sources: GOC:mah Also known as: positive regulation of histidyl-aspartyl phosphorelay, up regulation of two-component signal transduction, up-regulation of two-component signal transduction, upregulation of two-component signal transduction, activation of two-component signal transduction, positive regulation of two-component signal transduction system (phosphorelay), stimulation of two-component signal transduction